inhibitory synapse assembly [GO:1904862] (BP) Relationships: is a type of GO:0007416 Also known as: inhibitory synapse formation Definition: The aggregation, arrangement and bonding together of a set of components to form an inhibitory synapse. Regulation: regulated by GO:1905702; negatively regulated by negative regulation of inhibitory synapse assembly [GO:1905703]; positively regulated by positive regulation of inhibitory synapse assembly [GO:1905704] Sources: GOC:PARL, GOC:TermGenie, GOC:bf, GO_REF:0000079